{
  "gene": "UniProtKB:O14792",
  "gene_name": "Heparan sulfate glucosamine 3-O-sulfotransferase 1",
  "term_id": "GO:0008467",
  "term_label": "[heparan sulfate]-glucosamine 3-sulfotransferase activity",
  "gene_symbol": "HS3ST1"
}